{
  "term_label": "endoplasmic reticulum",
  "gene_name": "E3 ubiquitin-protein ligase RNF133",
  "gene": "UniProtKB:Q8WVZ7",
  "term_id": "GO:0005783",
  "gene_symbol": "RNF133"
}